{
  "gene_symbol": "FAM184A",
  "term_label": "Unknown biological process",
  "gene_name": "Protein FAM184A",
  "gene": "UniProtKB:Q8NB25",
  "term_id": "UNKNOWN:0002"
}